{
  "term_label": "Unknown molecular function",
  "gene_name": "Spondin-2",
  "term_id": "UNKNOWN:0001",
  "gene_symbol": "SPON2",
  "gene": "UniProtKB:Q9BUD6"
}